regulation of female pigmentation [GO:0048089] (biological process) Sources: GOC:jid Definition: Any process that modulates the frequency, rate or extent of establishment of a pattern of pigment in females. Relationships: is a type of regulation of developmental pigmentation [GO:0048070]; is a type of regulation of developmental process [GO:0050793]; is a type of GO:2000241; regulates female pigmentation [GO:0048095] Subtypes: GO:0048090, positive regulation of female pigmentation [GO:0048091]